{
  "gene": "UniProtKB:A0A0G2JN53",
  "term_id": "UNKNOWN:0003",
  "gene_symbol": "A0A0G2JN53",
  "gene_name": "IQ motif and SEC7 domain-containing protein 3",
  "term_label": "Unknown cellular component"
}